foregut morphogenesis [GO:0007440] (biological process) Relationships: is a type of GO:0009653; is part of GO:0048546 Sources: GOC:jid Definition: The process in which the anatomical structures of the foregut are generated and organized.